{
  "term_id": "GO:0007229",
  "gene_symbol": "ITGA11",
  "gene": "UniProtKB:Q9UKX5",
  "gene_name": "Integrin alpha-11",
  "term_label": "integrin-mediated signaling pathway"
}